{
  "term_label": "mitochondrion",
  "term_id": "GO:0005739",
  "gene_symbol": "SDHAF1",
  "gene": "UniProtKB:A6NFY7",
  "gene_name": "Succinate dehydrogenase assembly factor 1, mitochondrial"
}